{
  "gene": "UniProtKB:O60716",
  "gene_name": "Catenin delta-1",
  "gene_symbol": "CTNND1",
  "term_id": "GO:0005634",
  "term_label": "nucleus"
}